3-beta-hydroxysteroid 3-dehydrogenase (NADP+) activity [GO:0000253] (molecular function) Relationships: is a type of steroid dehydrogenase activity, acting on the CH-OH group of donors, NAD or NADP as acceptor [GO:0033764] Also known as: 3-keto sterol reductase activity, 3-keto-steroid reductase activity, 3-KSR activity, 3beta-hydroxy-steroid:NADP+ 3-oxidoreductase References: PMID:9811880 Sources: EC:1.1.1.270, GOC:mah Definition: Catalysis of the reaction: a 3-betahydroxyl sterol + NADP+ = a 3-oxosterol sterol + NADPH + H+.